negative regulation of protein secretion [GO:0050709] (biological process) Definition: Any process that stops, prevents, or reduces the frequency, rate or extent of the controlled release of a protein from a cell. Also known as: down regulation of protein secretion, down-regulation of protein secretion, downregulation of protein secretion, inhibition of protein secretion Subtypes: negative regulation of insulin secretion [GO:0046676], negative regulation of Wnt protein secretion [GO:0061358], GO:0070164, negative regulation of secretion of lysosomal enzymes [GO:0090341], negative regulation of renin secretion into blood stream [GO:1900134], GO:1902277, negative regulation of prolactin secretion [GO:1902721], GO:1904243, negative regulation of matrix metallopeptidase secretion [GO:1904465], GO:2001285 Sources: GOC:ai Relationships: is_a regulation of protein secretion [GO:0050708]; is a type of GO:0051224; is a type of negative regulation of secretion by cell [GO:1903531]; negatively regulates protein secretion [GO:0009306]